{
  "gene_name": "Golgi SNAP receptor complex member 2",
  "term_label": "SNARE binding",
  "term_id": "GO:0000149",
  "gene_symbol": "GOSR2",
  "gene": "UniProtKB:O14653"
}